oligogalacturonide transport [GO:0033156] (biological process) Definition: The directed movement of oligogalacturonides into, out of or within a cell, or between cells, by means of some agent such as a transporter or pore. Relationships: is a type of GO:0015772 Sources: GOC:mlg